vitamin transmembrane transport [GO:0035461] (biological process) Note: Note that this term is not intended for use in annotating lateral movement within membranes. Definition: The process in which a vitamin is transported across a membrane. A vitamin is one of a number of unrelated organic substances that occur in many foods in small amounts and that are necessary in trace amounts for the normal metabolic functioning of the body. Relationships: is a type of vitamin transport [GO:0051180]; is a type of transmembrane transport [GO:0055085] Subtypes: L-ascorbic acid transmembrane transport [GO:0015882], pantothenate transmembrane transport [GO:0015887], thiamine transmembrane transport [GO:0071934], vitamin A import into cell [GO:0071939], folate transmembrane transport [GO:0098838], pyridoxal transmembrane transport [GO:1903090], pyridoxamine transmembrane transport [GO:1903091], pyridoxine transmembrane transport [GO:1903092], biotin import across plasma membrane [GO:1905135] Also known as: vitamin membrane transport Sources: GOC:bf